{
  "gene": "UniProtKB:A6NDY2",
  "gene_symbol": "FAM90A10",
  "term_id": "UNKNOWN:0002",
  "term_label": "Unknown biological process",
  "gene_name": "Putative protein FAM90A10"
}